{
  "term_id": "GO:0042147",
  "gene_symbol": "VPS29",
  "gene": "UniProtKB:Q9UBQ0",
  "gene_name": "Vacuolar protein sorting-associated protein 29",
  "term_label": "retrograde transport, endosome to Golgi"
}